{
  "term_id": "GO:0005886",
  "gene_name": "Angiotensin-converting enzyme",
  "gene": "UniProtKB:P12821",
  "term_label": "plasma membrane",
  "gene_symbol": "ACE"
}